{
  "gene_name": "Leucine zipper protein 4",
  "term_label": "Unknown biological process",
  "gene_symbol": "LUZP4",
  "gene": "UniProtKB:Q9P127",
  "term_id": "UNKNOWN:0002"
}